{
  "gene": "UniProtKB:P10523",
  "term_id": "GO:0007600",
  "gene_symbol": "SAG",
  "term_label": "sensory perception",
  "gene_name": "S-arrestin"
}